mating behavior [GO:0007617] (biological process) Also known as: mating behaviour Definition: The behavioral interactions between organisms for the purpose of mating, or sexual reproduction resulting in the formation of zygotes. Sources: GOC:ai, GOC:dph Subtypes: courtship behavior [GO:0007619], copulation [GO:0007620], GO:0035648, mating behavior, sex discrimination [GO:0048047], GO:0060179, female mating behavior [GO:0060180] Relationships: is a type of reproductive behavior [GO:0019098]